ripoptosome assembly involved in necroptotic process [GO:1901026] (biological process) Regulation: regulated by regulation of ripoptosome assembly involved in necroptotic process [GO:1902442]; negatively regulated by negative regulation of ripoptosome assembly involved in necroptotic process [GO:1902443] Also known as: ripoptosome assembly involved in necroptosis Definition: The aggregation, arrangement and bonding together of ripoptosome components leading to a necroptotic process. Relationships: is a type of ripoptosome assembly [GO:0097343]; is part of GO:0070266 References: PMID:22274400 Sources: GOC:TermGenie, GOC:mtg_apoptosis